shorthand [oboInOwl#shorthand]